symbiont-mediated suppression of host JAK-STAT cascade via inhibition of JAK1 activity [GO:0039576] (biological process) Also known as: disruption by virus of host JAK-STAT cascade via inhibition of JAK1 activity, inhibition of host JAK activity by virus, negative regulation by virus of host JAK, negative regulation by virus of tyrosine phosphorylation of host STAT protein, suppression by virus of host JAK-STAT cascade via inhibition of JAK1 activity, suppression by virus of host JAK1 activity, suppression by virus of tyrosine phosphorylation of host STAT protein, viral inhibition of tyrosine phosphorylation of host STAT protein Definition: A process in which a symbiont interferes with, inhibits or disrupt a JAK-STAT signal cascade in the host organism by reducing the activity of host JAK1 (Janus Kinase 1). References: PMID:16188985 Relationships: is a type of symbiont-mediated suppression of host JAK-STAT cascade [GO:0039514] Note: This term is for annotation of symbiont proteins that counteract the host innate immune response.